{
  "gene_name": "Regulator of G-protein signaling 7",
  "gene_symbol": "RGS7",
  "gene": "UniProtKB:P49802",
  "term_label": "GTPase activator activity",
  "term_id": "GO:0005096"
}